{
  "gene_symbol": "POLR3B",
  "gene_name": "DNA-directed RNA polymerase III subunit RPC2",
  "term_id": "GO:0042796",
  "gene": "UniProtKB:Q9NW08",
  "term_label": "snRNA transcription by RNA polymerase III"
}